{
  "gene_symbol": "CYP1A1",
  "gene_name": "Cytochrome P450 1A1",
  "term_id": "GO:0005739",
  "gene": "UniProtKB:P04798",
  "term_label": "mitochondrion"
}